{
  "term_id": "GO:0006629",
  "term_label": "lipid metabolic process",
  "gene_name": "Leptin",
  "gene_symbol": "LEP",
  "gene": "UniProtKB:P41159"
}